{
  "gene_name": "Cytosolic acyl coenzyme A thioester hydrolase",
  "term_label": "cytosol",
  "term_id": "GO:0005829",
  "gene_symbol": "ACOT7",
  "gene": "UniProtKB:O00154"
}